G1/S transition of mitotic cell cycle [GO:0000082] (biological process) Regulation: positively regulated by positive regulation of G1/S transition of mitotic cell cycle [GO:1900087]; regulated by regulation of G1/S transition of mitotic cell cycle [GO:2000045]; negatively regulated by negative regulation of G1/S transition of mitotic cell cycle [GO:2000134] Relationships: is a type of mitotic cell cycle phase transition [GO:0044772]; is a type of cell cycle G1/S phase transition [GO:0044843] Definition: The mitotic cell cycle transition by which a cell in G1 commits to S phase. The process begins with the build up of G1 cyclin-dependent kinase (G1 CDK), resulting in the activation of transcription of G1 cyclins. The process ends with the positive feedback of the G1 cyclins on the G1 CDK which commits the cell to S phase, in which DNA replication is initiated. Sources: GOC:mtg_cell_cycle